{
  "term_id": "UNKNOWN:0003",
  "term_label": "Unknown cellular component",
  "gene_name": "LYR motif-containing protein 9",
  "gene": "UniProtKB:A8MSI8",
  "gene_symbol": "LYRM9"
}